{
  "term_label": "calcium ion binding",
  "gene": "UniProtKB:Q9UM19",
  "gene_name": "Hippocalcin-like protein 4",
  "gene_symbol": "HPCAL4",
  "term_id": "GO:0005509"
}